{
  "term_id": "GO:0008320",
  "gene_name": "TOMM20-like protein 1",
  "gene": "UniProtKB:Q6UXN7",
  "gene_symbol": "TOMM20L",
  "term_label": "protein transmembrane transporter activity"
}